transforming growth factor beta receptor activity, type II [GO:0005026] (molecular function) Sources: GOC:mah Definition: Combining with transforming growth factor beta to initiate a change in cell activity; upon ligand binding, binds to and catalyzes the phosphorylation of a type I TGF-beta receptor. Also known as: type II TGF-beta receptor activity, type II TGFbeta receptor activity, type II transforming growth factor beta receptor activity, transforming growth factor beta ligand binding to type II receptor Relationships: is a type of transforming growth factor beta receptor activity [GO:0005024]; has part transforming growth factor beta binding [GO:0050431]